{
  "term_id": "GO:0032755",
  "gene_name": "Toll-like receptor 7",
  "gene": "UniProtKB:Q9NYK1",
  "term_label": "positive regulation of interleukin-6 production",
  "gene_symbol": "TLR7"
}